{
  "term_label": "cytoplasm",
  "gene_name": "Serine_threonine-protein kinase TAO2",
  "gene": "UniProtKB:Q9UL54",
  "term_id": "GO:0005737",
  "gene_symbol": "TAOK2"
}